{
  "term_id": "GO:0008503",
  "gene_symbol": "GABRA3",
  "gene": "UniProtKB:P34903",
  "term_label": "benzodiazepine receptor activity",
  "gene_name": "Gamma-aminobutyric acid receptor subunit alpha-3"
}